{
  "gene": "UniProtKB:Q9H7Y0",
  "term_label": "Unknown molecular function",
  "term_id": "UNKNOWN:0001",
  "gene_symbol": "DIPK2B",
  "gene_name": "Divergent protein kinase domain 2B"
}